modification-dependent protein catabolic process [GO:0019941] (biological process) Sources: GOC:go_curators Subtypes: ubiquitin-dependent protein catabolic process [GO:0006511], GO:0030327, oxidation-dependent protein catabolic process [GO:0070407] Also known as: modification-dependent protein breakdown, modification-dependent protein catabolism, modification-dependent protein degradation, modification-dependent proteolysis, modification-initiated protein catabolic process, modification-initiated protein catabolism, modification-initiated proteolysis, protein-ligand-dependent protein catabolic process, protein-ligand-dependent protein catabolism, protein degradation tagging activity Definition: The chemical reactions and pathways resulting in the breakdown of a protein or peptide by hydrolysis of its peptide bonds, initiated by the covalent modification of the target protein. Relationships: is a type of modification-dependent macromolecule catabolic process [GO:0043632]; is a type of proteolysis involved in protein catabolic process [GO:0051603]; has part protein modification process [GO:0036211]